positive regulation of epithelial cell proliferation involved in prostate gland development [GO:0060769] (BP) Sources: GOC:dph Relationships: is a type of positive regulation of epithelial cell proliferation [GO:0050679]; is a type of positive regulation of developmental process [GO:0051094]; is a type of GO:0060768; is a type of positive regulation of reproductive process [GO:2000243]; positively regulates epithelial cell proliferation involved in prostate gland development [GO:0060767] Definition: Any process that increases the rate, frequency or extent of epithelial cell proliferation that contributes to the progression of the prostate gland over time.